{
  "gene_symbol": "ZNF620",
  "gene_name": "Zinc finger protein 620",
  "term_id": "GO:0005634",
  "term_label": "nucleus",
  "gene": "UniProtKB:Q6ZNG0"
}